{
  "term_id": "GO:0042742",
  "gene": "UniProtKB:P10645",
  "gene_name": "Chromogranin-A",
  "gene_symbol": "CHGA",
  "term_label": "defense response to bacterium"
}